{
  "gene": "UniProtKB:Q9BZE4",
  "gene_symbol": "GTPBP4",
  "term_id": "GO:0005730",
  "gene_name": "GTP-binding protein 4",
  "term_label": "nucleolus"
}